{
  "gene": "UniProtKB:Q5TB30",
  "gene_symbol": "DEPDC1",
  "term_id": "GO:0005634",
  "term_label": "nucleus",
  "gene_name": "DEP domain-containing protein 1A"
}